viral RNA genome replication [GO:0039694] (biological process) Subtypes: negative stranded viral RNA replication [GO:0039689], GO:0039690, double stranded viral RNA replication [GO:0039691], single stranded viral RNA replication via double stranded DNA intermediate [GO:0039692] Definition: The replication of a viral RNA genome. Sources: GOC:bf, GOC:jl Regulation: regulated by host-mediated perturbation of viral RNA genome replication [GO:0044830] Relationships: is a type of viral genome replication [GO:0019079]; is a type of RNA biosynthetic process [GO:0032774]